Rad51B-Rad51C-Rad51D-XRCC2 complex [GO:0033063] (cellular component) Definition: A DNA recombinase mediator complex that contains the Rad51 paralogs RAD51B, RAD51C, RAD51D, and XRCC2, or orthologs thereof. References: PMID:16093548, PMID:17114795 Sources: GOC:mah Also known as: BCDX2 complex Relationships: is a type of DNA recombinase mediator complex [GO:0033061]; is a type of nuclear protein-containing complex [GO:0140513]